{
  "gene": "UniProtKB:P0DPH8",
  "term_id": "GO:0005525",
  "gene_symbol": "TUBA3D",
  "term_label": "GTP binding",
  "gene_name": "Tubulin alpha-3D chain"
}